{
  "gene_name": "Probable cation-transporting ATPase 13A5",
  "term_id": "GO:0031902",
  "gene_symbol": "ATP13A5",
  "gene": "UniProtKB:Q4VNC0",
  "term_label": "late endosome membrane"
}